{
  "term_id": "UNKNOWN:0001",
  "gene_symbol": "OR11H2",
  "gene_name": "Olfactory receptor 11H2",
  "term_label": "Unknown molecular function",
  "gene": "UniProtKB:Q8NH07"
}